{
  "gene_symbol": "TYR",
  "term_id": "GO:0042470",
  "term_label": "melanosome",
  "gene": "UniProtKB:P14679",
  "gene_name": "Tyrosinase"
}